{
  "term_id": "GO:0005814",
  "gene_name": "Cytosolic carboxypeptidase 3",
  "gene_symbol": "AGBL3",
  "gene": "UniProtKB:Q8NEM8",
  "term_label": "centriole"
}